phenylpropanoid biosynthetic process [GO:0009699] (biological process) Definition: The chemical reactions and pathways resulting in the formation of aromatic derivatives of trans-cinnamic acid. Subtypes: chalcone biosynthetic process [GO:0009715], isoflavonoid biosynthetic process [GO:0009717], cinnamic acid biosynthetic process [GO:0009800], cinnamic acid ester biosynthetic process [GO:0009802], GO:0009805, lignan biosynthetic process [GO:0009807], lignin biosynthetic process [GO:0009809], GO:0010023, suberin biosynthetic process [GO:0010345], GO:0033497, GO:0033525, eugenol biosynthetic process [GO:0042855] Sources: GOC:jl Also known as: phenylpropanoid anabolism, phenylpropanoid biosynthesis, phenylpropanoid formation, phenylpropanoid synthesis Relationships: is a type of phenylpropanoid metabolic process [GO:0009698]; is a type of secondary metabolite biosynthetic process [GO:0044550]